{
  "gene_symbol": "BRF1",
  "term_label": "RNA polymerase III type 3 promoter sequence-specific DNA binding",
  "gene": "UniProtKB:Q92994",
  "term_id": "GO:0001006",
  "gene_name": "Transcription factor IIIB 90 kDa subunit"
}